{
  "gene_name": "Ankyrin repeat and SAM domain-containing protein 6",
  "gene_symbol": "ANKS6",
  "term_id": "UNKNOWN:0001",
  "gene": "UniProtKB:Q68DC2",
  "term_label": "Unknown molecular function"
}